{
  "gene": "UniProtKB:O43734",
  "term_id": "UNKNOWN:0003",
  "term_label": "Unknown cellular component",
  "gene_symbol": "TRAF3IP2",
  "gene_name": "E3 ubiquitin ligase TRAF3IP2"
}